{
  "term_id": "GO:0003254",
  "gene_name": "Potassium_sodium hyperpolarization-activated cyclic nucleotide-gated channel 2",
  "gene": "UniProtKB:Q9UL51",
  "term_label": "regulation of membrane depolarization",
  "gene_symbol": "HCN2"
}